{
  "gene_symbol": "IGHV6-1",
  "gene_name": "Immunoglobulin heavy variable 6-1",
  "term_label": "antigen binding",
  "gene": "UniProtKB:A0A0B4J1U7",
  "term_id": "GO:0003823"
}